{
  "gene_name": "Rho GTPase-activating protein SYDE2",
  "gene_symbol": "SYDE2",
  "term_id": "GO:0046578",
  "gene": "UniProtKB:Q5VT97",
  "term_label": "regulation of Ras protein signal transduction"
}